{
  "term_label": "cadherin binding",
  "gene_symbol": "CTNND1",
  "gene": "UniProtKB:O60716",
  "term_id": "GO:0045296",
  "gene_name": "Catenin delta-1"
}